{
  "gene_symbol": "TTYH3",
  "term_id": "GO:0005886",
  "gene": "UniProtKB:Q9C0H2",
  "gene_name": "Protein tweety homolog 3",
  "term_label": "plasma membrane"
}